D-arabinose 1-dehydrogenase [NAD(P)+] activity [GO:0045290] (molecular function) Also known as: D-arabinose:NAD(P)+ 1-oxidoreductase activity Relationships: is a type of oxidoreductase activity, acting on the CH-OH group of donors, NAD or NADP as acceptor [GO:0016616] Definition: Catalysis of the reaction: D-arabinose + NAD(P)+ = D-arabinono-1,4-lactone + NAD(P)H + H+. Sources: EC:1.1.1.117 Subtypes: GO:0047816, D-arabinose 1-dehydrogenase (NADP+) activity [GO:0106271]